{
  "gene": "UniProtKB:Q96BZ9",
  "gene_name": "TBC1 domain family member 20",
  "term_label": "endoplasmic reticulum membrane",
  "term_id": "GO:0005789",
  "gene_symbol": "TBC1D20"
}